{
  "gene": "UniProtKB:Q8IWP9",
  "term_label": "Unknown cellular component",
  "term_id": "UNKNOWN:0003",
  "gene_symbol": "CCDC28A",
  "gene_name": "Coiled-coil domain-containing protein 28A"
}